{
  "term_label": "regulation of actin filament polymerization",
  "gene_symbol": "ARHGAP18",
  "term_id": "GO:0030833",
  "gene": "UniProtKB:Q8N392",
  "gene_name": "Rho GTPase-activating protein 18"
}